pyrimidine nucleobase catabolic process [GO:0006208] (biological process) Subtypes: cytosine catabolic process [GO:0006209], thymine catabolic process [GO:0006210], GO:0006212, pyrimidine nucleobase fermentation [GO:0043466] Sources: GOC:go_curators Definition: The chemical reactions and pathways resulting in the breakdown of pyrimidine nucleobases, 1,3-diazine, organic nitrogenous bases. Also known as: pyrimidine base breakdown, pyrimidine base catabolic process, pyrimidine base catabolism, pyrimidine base degradation Relationships: is a type of pyrimidine nucleobase metabolic process [GO:0006206]; is a type of nucleobase catabolic process [GO:0046113]; is a type of pyrimidine-containing compound catabolic process [GO:0072529]